{
  "term_label": "Rho protein signal transduction",
  "gene_name": "Uncharacterized protein C15orf62, mitochondrial",
  "term_id": "GO:0007266",
  "gene": "UniProtKB:A8K5M9",
  "gene_symbol": "C15orf62"
}